{
  "term_id": "GO:0014069",
  "term_label": "postsynaptic density",
  "gene_symbol": "ADGRB1",
  "gene": "UniProtKB:O14514",
  "gene_name": "Adhesion G protein-coupled receptor B1"
}